{
  "term_label": "plasma membrane",
  "gene": "UniProtKB:Q6T4P5",
  "gene_name": "Phospholipid phosphatase-related protein type 3",
  "term_id": "GO:0005886",
  "gene_symbol": "PLPPR3"
}